{
  "term_label": "external side of plasma membrane",
  "gene": "UniProtKB:P07766",
  "gene_name": "T-cell surface glycoprotein CD3 epsilon chain",
  "term_id": "GO:0009897",
  "gene_symbol": "CD3E"
}